{
  "gene_name": "Transcription factor 15",
  "gene": "UniProtKB:Q12870",
  "term_id": "UNKNOWN:0003",
  "gene_symbol": "TCF15",
  "term_label": "Unknown cellular component"
}